{
  "term_id": "GO:0050291",
  "gene_symbol": "TLCD3B",
  "gene": "UniProtKB:Q71RH2",
  "term_label": "sphingosine N-acyltransferase activity",
  "gene_name": "Ceramide synthase"
}